{
  "gene_name": "Inactive rhomboid protein 2",
  "term_label": "Unknown molecular function",
  "term_id": "UNKNOWN:0001",
  "gene_symbol": "RHBDF2",
  "gene": "UniProtKB:Q6PJF5"
}